{
  "term_id": "GO:0060326",
  "gene_symbol": "CX3CR1",
  "gene_name": "CX3C chemokine receptor 1",
  "gene": "UniProtKB:P49238",
  "term_label": "cell chemotaxis"
}